septal periplasm [GO:0036240] (cellular component) Relationships: is a type of periplasmic space [GO:0042597] References: PMID:21564341 Sources: GOC:di Also known as: cell wall-enclosed septal periplasm Definition: The region between the plasma membrane and the cell wall, as found in organisms such as filamentous fungi.